{
  "term_label": "nucleus",
  "gene": "UniProtKB:Q9NWW7",
  "gene_symbol": "C2orf42",
  "term_id": "GO:0005634",
  "gene_name": "Uncharacterized protein C2orf42"
}